mitochondrial endopeptidase Clp complex [GO:0009841] (cellular component) Sources: GOC:mah Relationships: is a type of endopeptidase Clp complex [GO:0009368]; is a type of mitochondrial protein-containing complex [GO:0098798]; is part of mitochondrial matrix [GO:0005759] Definition: A Clp endopeptidase complex located in the mitochondrion.